{
  "term_label": "de novo centriole assembly involved in multi-ciliated epithelial cell differentiation",
  "term_id": "GO:0098535",
  "gene_name": "Centrosomal protein of 63 kDa",
  "gene": "UniProtKB:Q96MT8",
  "gene_symbol": "CEP63"
}